{
  "term_label": "regulation of dendrite morphogenesis",
  "gene": "UniProtKB:P46934",
  "gene_symbol": "NEDD4",
  "term_id": "GO:0048814",
  "gene_name": "E3 ubiquitin-protein ligase NEDD4"
}